{
  "gene_name": "Immunoglobulin heavy variable 3-30-5",
  "gene": "UniProtKB:P0DP03",
  "term_id": "GO:0003823",
  "term_label": "antigen binding",
  "gene_symbol": "IGHV3-30-5"
}